{
  "gene": "UniProtKB:Q8NHB7",
  "gene_symbol": "OR5K1",
  "term_id": "GO:0005549",
  "gene_name": "Olfactory receptor 5K1",
  "term_label": "odorant binding"
}